{
  "term_id": "GO:0043138",
  "gene_name": "DNA replication licensing factor MCM2",
  "term_label": "3'-5' DNA helicase activity",
  "gene": "UniProtKB:P49736",
  "gene_symbol": "MCM2"
}